{
  "gene_symbol": "NALCN",
  "gene": "UniProtKB:Q8IZF0",
  "term_label": "positive regulation of synaptic transmission, cholinergic",
  "gene_name": "Sodium leak channel NALCN",
  "term_id": "GO:0032224"
}